{
  "gene_symbol": "FAM90A22",
  "term_label": "Unknown cellular component",
  "gene_name": "Putative protein FAM90A22",
  "gene": "UniProtKB:A8MWA6",
  "term_id": "UNKNOWN:0003"
}